{
  "gene_symbol": "OR5H1",
  "gene": "UniProtKB:A6NKK0",
  "term_label": "Unknown biological process",
  "term_id": "UNKNOWN:0002",
  "gene_name": "Olfactory receptor 5H1"
}